{
  "term_id": "GO:0003341",
  "gene": "UniProtKB:Q5TD94",
  "gene_symbol": "RSPH4A",
  "term_label": "cilium movement",
  "gene_name": "Radial spoke head protein 4 homolog A"
}